myeloid leukocyte differentiation [GO:0002573] (biological process) Relationships: is a type of leukocyte differentiation [GO:0002521]; is a type of myeloid cell differentiation [GO:0030099] Subtypes: GO:0030224, macrophage differentiation [GO:0030225], osteoclast differentiation [GO:0030316], GO:0030851, myeloid dendritic cell differentiation [GO:0043011], mast cell differentiation [GO:0060374], mature conventional dendritic cell differentiation [GO:0097029] Definition: The process in which a relatively unspecialized myeloid precursor cell acquires the specialized features of any cell of the myeloid leukocyte lineage. Regulation: RO_0002211 by regulation of myeloid leukocyte differentiation [GO:0002761]; negatively regulated by negative regulation of myeloid leukocyte differentiation [GO:0002762]; positively regulated by GO:0002763 References: PMID:16551251 Sources: GOC:add Also known as: myeloid leucocyte differentiation